{
  "gene_name": "Transcription factor SPT20 homolog-like 1",
  "term_label": "regulation of transcription by RNA polymerase II",
  "gene_symbol": "SUPT20HL1",
  "gene": "UniProtKB:Q3ZLR7",
  "term_id": "GO:0006357"
}